positive regulation of lamellipodium organization [GO:1902745] (biological process) References: PMID:16054028 Sources: GOC:TermGenie, GOC:als, GO_REF:0000058 Subtypes: positive regulation of lamellipodium assembly [GO:0010592], GO:2000394 Relationships: is a type of GO:0031346; is_a regulation of lamellipodium organization [GO:1902743]; positively regulates GO:0097581 Also known as: up regulation of lamellipodium organization, up-regulation of lamellipodium organization, upregulation of lamellipodium organization, activation of lamellipodium organization Definition: Any process that activates or increases the frequency, rate or extent of lamellipodium organization.